{
  "gene_symbol": "CUTC",
  "term_label": "Unknown biological process",
  "gene_name": "Copper homeostasis protein cutC homolog",
  "gene": "UniProtKB:Q9NTM9",
  "term_id": "UNKNOWN:0002"
}